{
  "gene_symbol": "ZPR1",
  "gene_name": "Zinc finger protein ZPR1",
  "gene": "UniProtKB:O75312",
  "term_label": "Cajal body organization",
  "term_id": "GO:0030576"
}